transmembrane transporter activity [GO:0022857] (molecular function) Definition: Enables the transfer of a substance, usually a specific substance or a group of related substances, from one side of a membrane to the other. Relationships: is a type of transporter activity [GO:0005215]; is part of transmembrane transport [GO:0055085] Also known as: substrate-specific transmembrane transporter activity, substrate-specific transporter activity, uptake permease activity, uptake transmembrane transporter activity Sources: GOC:jid, GOC:mtg_transport, ISBN:0815340729 Subtypes: amine transmembrane transporter activity [GO:0005275], neurotransmitter transmembrane transporter activity [GO:0005326], water transmembrane transporter activity [GO:0005372], chlorophyll catabolite transmembrane transporter activity [GO:0010290], monoatomic ion transmembrane transporter activity [GO:0015075], aluminum ion transmembrane transporter activity [GO:0015083], molybdate ion transmembrane transporter activity [GO:0015098], antimonite transmembrane transporter activity [GO:0015104], GO:0015105, bicarbonate transmembrane transporter activity [GO:0015106], GO:0015107, chromate transmembrane transporter activity [GO:0015109], cyanate transmembrane transporter activity [GO:0015110], nitrate transmembrane transporter activity [GO:0015112], nitrite transmembrane transporter activity [GO:0015113], silicate transmembrane transporter activity [GO:0015115], mevalonate transmembrane transporter activity [GO:0015130], carbohydrate transmembrane transporter activity [GO:0015144], polyol transmembrane transporter activity [GO:0015166], amino acid transmembrane transporter activity [GO:0015171], polyamine transmembrane transporter activity [GO:0015203], nucleobase transmembrane transporter activity [GO:0015205], choline transmembrane transporter activity [GO:0015220], biopterin transmembrane transporter activity [GO:0015224], GO:0015232, bicyclomycin transmembrane transporter activity [GO:0015545], 3-hydroxyphenyl propanoate transmembrane transporter activity [GO:0015551], efflux transmembrane transporter activity [GO:0015562], alkane transmembrane transporter activity [GO:0015567], iron chelate transmembrane transporter activity [GO:0015603], organophosphate ester transmembrane transporter activity [GO:0015605], ferric triacetylfusarinine C transmembrane transporter activity [GO:0015621], quaternary ammonium group transmembrane transporter activity [GO:0015651], tellurite transmembrane transporter activity [GO:0015654], alcohol transmembrane transporter activity [GO:0015665], GO:0015932, oxidative phosphorylation uncoupler activity [GO:0017077], toxin transmembrane transporter activity [GO:0019534], passive transmembrane transporter activity [GO:0022803], active transmembrane transporter activity [GO:0022804], mobile ion carrier activity [GO:0022809], macromolecule transmembrane transporter activity [GO:0022884], nitric oxide transmembrane transporter activity [GO:0030184], pyridoxal transmembrane transporter activity [GO:0031925], pyridoxamine transmembrane transporter activity [GO:0031927], GO:0031928, carbon dioxide transmembrane transporter activity [GO:0035379], amide transmembrane transporter activity [GO:0042887], xenobiotic transmembrane transporter activity [GO:0042910], carboxylic acid transmembrane transporter activity [GO:0046943], chromium ion transmembrane transporter activity [GO:0070835], modified amino acid transmembrane transporter activity [GO:0072349], GO:0080161, vitamin transmembrane transporter activity [GO:0090482], GO:0160283, ergothioneine transmembrane transporter activity [GO:0170001], lipoate transmembrane transporter activity [GO:0170004], lipid transmembrane transporter activity [GO:0170055], acetate ester transmembrane transporter activity [GO:1901375], azole transmembrane transporter activity [GO:1901474], carbohydrate derivative transmembrane transporter activity [GO:1901505], lipo-chitin oligosaccharide transmembrane transporter activity [GO:1901513], GO:1901515, sulfur compound transmembrane transporter activity [GO:1901682], arsenate ion transmembrane transporter activity [GO:1901683], GO:1901702, peptide transmembrane transporter activity [GO:1904680] Regulation: regulated by GO:0022898